{
  "gene_name": "Leucine-rich repeat-containing protein 27",
  "term_label": "Unknown cellular component",
  "gene_symbol": "LRRC27",
  "term_id": "UNKNOWN:0003",
  "gene": "UniProtKB:Q9C0I9"
}